{
  "term_label": "central nervous system myelination",
  "gene": "UniProtKB:Q13491",
  "gene_symbol": "GPM6B",
  "gene_name": "Neuronal membrane glycoprotein M6-b",
  "term_id": "GO:0022010"
}